negative regulation of alkane biosynthetic process [GO:1901578] (biological process) Definition: Any process that stops, prevents or reduces the frequency, rate or extent of alkane biosynthetic process. Also known as: down regulation of alkane anabolism, down regulation of alkane biosynthesis, down regulation of alkane biosynthetic process, down regulation of alkane formation, down regulation of alkane synthesis, down-regulation of alkane anabolism, down-regulation of alkane biosynthesis, down-regulation of alkane biosynthetic process, down-regulation of alkane formation, down-regulation of alkane synthesis, downregulation of alkane anabolism, downregulation of alkane biosynthesis, downregulation of alkane biosynthetic process, downregulation of alkane formation, downregulation of alkane synthesis, inhibition of alkane anabolism, inhibition of alkane biosynthesis, inhibition of alkane formation, inhibition of alkane synthesis, negative regulation of alkane anabolism, negative regulation of alkane biosynthesis, negative regulation of alkane formation, negative regulation of alkane synthesis, inhibition of alkane biosynthetic process Relationships: is_a GO:0009890; is a type of regulation of alkane biosynthetic process [GO:1901577]; negatively regulates GO:0043447 Subtypes: GO:1900319, negative regulation of methane biosynthetic process from trimethylamine [GO:1900331], negative regulation of methane biosynthetic process from 3-(methylthio)propionic acid [GO:1900334], negative regulation of methane biosynthetic process from carbon monoxide [GO:1900337], negative regulation of methane biosynthetic process from formic acid [GO:1900340], GO:1900343, negative regulation of methane biosynthetic process from methanethiol [GO:1900346], negative regulation of methane biosynthetic process from methylamine [GO:1900349], negative regulation of tridecane biosynthetic process [GO:1900885], negative regulation of pentadecane biosynthetic process [GO:1900888], negative regulation of heptadecane biosynthetic process [GO:1900897] Sources: GOC:TermGenie